structural constituent of collagen and cuticulin-based cuticle [GO:0042329] (molecular function) Relationships: is a type of structural constituent of cuticle [GO:0042302] Sources: GOC:jl, GOC:mtg_sensu Definition: The action of a molecule that contributes to the structural integrity of a collagen and cuticulin-based cuticle. An example of this process is found in Caenorhabditis elegans. Also known as: structural constituent of cuticle